APC-tubulin-IQGAP1 complex [GO:0034741] (cellular component) Note: Note that the gene/protein name 'APC' should not be confused with the abbreviation for 'anaphase promoting complex'. Also known as: 60S APC complex Definition: A protein complex that contains the tumor suppressor protein adenomatous polyposis coli (APC), alpha-tubulin, gamma-tubulin, and the Rac1 and Cdc42 effector IQGAP1; may play a role in cytoskeleton organization. References: PMID:17126424 Relationships: is a type of intracellular protein-containing complex [GO:0140535]; is a type of GO:1905360